{
  "gene_symbol": "MED18",
  "gene": "UniProtKB:Q9BUE0",
  "term_id": "GO:0070847",
  "gene_name": "Mediator of RNA polymerase II transcription subunit 18",
  "term_label": "core mediator complex"
}